{
  "term_id": "GO:0003730",
  "term_label": "mRNA 3'-UTR binding",
  "gene": "UniProtKB:Q96DU9",
  "gene_name": "Polyadenylate-binding protein 5",
  "gene_symbol": "PABPC5"
}